{
  "term_label": "dynein heavy chain binding",
  "term_id": "GO:0045504",
  "gene_name": "Dynein axonemal light chain 1",
  "gene_symbol": "DNAL1",
  "gene": "UniProtKB:Q4LDG9"
}